{
  "gene": "UniProtKB:Q8IZH2",
  "gene_name": "5'-3' exoribonuclease 1",
  "term_id": "GO:0016075",
  "term_label": "rRNA catabolic process",
  "gene_symbol": "XRN1"
}